{
  "term_id": "GO:0038023",
  "term_label": "signaling receptor activity",
  "gene_symbol": "CHAD",
  "gene_name": "Chondroadherin",
  "gene": "UniProtKB:O15335"
}